rhamnogalacturonan I biosynthetic process [GO:0010246] (biological process) Relationships: is a type of rhamnogalacturonan I metabolic process [GO:0010395]; is a type of cell wall polysaccharide biosynthetic process [GO:0070592] Also known as: rhamnogalacturonan I anabolism, rhamnogalacturonan I biosynthesis, rhamnogalacturonan I formation, rhamnogalacturonan I synthesis Sources: GOC:pz Definition: The chemical reactions and pathways resulting in the formation of rhamnogalacturonan I component of pectin, a rhamnose-rich pectic polysaccharide.